{
  "gene_name": "GRB2-associated-binding protein 2",
  "gene": "UniProtKB:Q9UQC2",
  "term_id": "GO:0007165",
  "gene_symbol": "GAB2",
  "term_label": "signal transduction"
}